protein localization to new growing cell tip [GO:1904758] (biological process) Relationships: is a type of protein localization to growing cell tip [GO:1902486] References: PMID:19431238 Sources: GOC:TermGenie, GO_REF:0000087 Also known as: protein localisation in new growing cell tip, protein localisation to new growing cell tip, protein localization in new growing cell tip, protein localization to new cell tip after activation of bipolar cell growth, protein localization to new growing cell end, protein localization to post-NETO new cell end, protein localization to post-NETO new cell tip, protein localization to post-new end take-off new cell tip Definition: A process in which a protein is transported to, or maintained in, a location within a new growing cell tip.